{
  "term_label": "actin filament binding",
  "gene_name": "Formin-like protein 1",
  "gene_symbol": "FMNL1",
  "gene": "UniProtKB:O95466",
  "term_id": "GO:0051015"
}